{
  "gene_symbol": "STK11",
  "term_id": "GO:0030010",
  "gene": "UniProtKB:Q15831",
  "term_label": "establishment of cell polarity",
  "gene_name": "Serine_threonine-protein kinase STK11"
}